regulation of ribosomal small subunit export from nucleus [GO:2000206] (biological process) Definition: Any process that modulates the frequency, rate or extent of ribosomal small subunit export from nucleus. Sources: GOC:mah Also known as: regulation of ribosomal small subunit export from cell nucleus, regulation of ribosomal small subunit export out of nucleus, regulation of ribosomal small subunit transport from nucleus to cytoplasm, regulation of ribosomal small subunit-nucleus export, regulation of 30S ribosomal subunit export from nucleus, regulation of 40S ribosomal subunit export from nucleus Relationships: is a type of GO:2000200; regulates ribosomal small subunit export from nucleus [GO:0000056] Subtypes: GO:2000207, positive regulation of ribosomal small subunit export from nucleus [GO:2000208]